{
  "gene_name": "Putative uncharacterized protein C6orf52",
  "term_label": "Unknown cellular component",
  "gene": "UniProtKB:Q5T4I8",
  "term_id": "UNKNOWN:0003",
  "gene_symbol": "C6orf52"
}